positive regulation of lung ciliated cell differentiation [GO:1901248] (biological process) Definition: Any process that activates or increases the frequency, rate or extent of lung ciliated cell differentiation. Sources: GOC:BHF, GOC:TermGenie Relationships: is a type of positive regulation of epithelial cell differentiation [GO:0030858]; is a type of GO:0051240; is a type of regulation of lung ciliated cell differentiation [GO:1901246]; RO_0002213 lung ciliated cell differentiation [GO:0061141] Also known as: up regulation of lung ciliated cell differentiation, up-regulation of lung ciliated cell differentiation, upregulation of lung ciliated cell differentiation, activation of lung ciliated cell differentiation